(1->4)-alpha-glucan biosynthetic process [GO:0070630] (biological process) Definition: The chemical reactions and pathways resulting in the formation of (1->4)-alpha-glucans, compounds composed of glucose residues linked by (1->4)-alpha-D-glucosidic bonds. Sources: GOC:mah Also known as: (1->4)-alpha-D-glucan anabolism, (1->4)-alpha-D-glucan biosynthesis, (1->4)-alpha-D-glucan formation, (1->4)-alpha-D-glucan synthesis, 1,4-alpha-glucan anabolism, 1,4-alpha-glucan biosynthesis, 1,4-alpha-glucan biosynthetic process, 1,4-alpha-glucan formation, 1,4-alpha-glucan synthesis, alpha-1,4 glucan anabolism, alpha-1,4 glucan biosynthesis, alpha-1,4 glucan biosynthetic process, alpha-1,4 glucan formation, alpha-1,4 glucan synthesis Relationships: is a type of GO:0030979; is a type of (1->4)-alpha-glucan metabolic process [GO:0070629]